intraciliary transport particle B [GO:0030992] (cellular component) Note: Note that we deem cilia and microtubule-based flagella to be equivalent. Also known as: intraflagellar transport complex B, intraflagellar transport particle B, IFT B complex, IFT complex B References: PMID:14570576, PMID:19253336 Sources: GOC:cilia, GOC:kmv Relationships: is a type of protein-containing complex [GO:0032991]; is part of GO:0030990 Definition: The larger subcomplex of the intraciliary transport particle; characterized complexes have molecular weights around 550 kDa.